{
  "term_id": "GO:0005615",
  "gene_symbol": "SERPINA1",
  "gene_name": "Alpha-1-antitrypsin",
  "term_label": "extracellular space",
  "gene": "UniProtKB:P01009"
}